SUMO activating enzyme activity [GO:0019948] (molecular function) Definition: Catalysis of the activation of the proteolytically processed small ubiquitin-related modifier SUMO, through the formation of an ATP-dependent high-energy thiolester bond. Also known as: SMT3 activating enzyme, SUMO E1 activator enzyme References: PMID:10187858, PMID:11265250 Sources: GOC:rn Relationships: is a type of ubiquitin-like modifier activating enzyme activity [GO:0008641]